{
  "term_label": "plasma membrane",
  "term_id": "GO:0005886",
  "gene_symbol": "EQTN",
  "gene": "UniProtKB:Q9NQ60",
  "gene_name": "Equatorin"
}